{
  "term_label": "nuclear speck",
  "gene": "UniProtKB:Q08170",
  "gene_name": "Serine_arginine-rich splicing factor 4",
  "gene_symbol": "SRSF4",
  "term_id": "GO:0016607"
}